{
  "gene_name": "Zinc finger protein 182",
  "term_id": "GO:0005634",
  "term_label": "nucleus",
  "gene_symbol": "ZNF182",
  "gene": "UniProtKB:P17025"
}